alveolar lamellar body [GO:0097208] (cellular component) Relationships: is_a GO:0042599 Sources: GOC:cjm, Wikipedia:Lamellar_granule Definition: A specialized secretory organelle found in type II pneumocytes and involved in the synthesis, secretion, and reutilization of pulmonary surfactant.